negative regulation of ruffle assembly [GO:1900028] (biological process) Definition: Any process that stops, prevents or reduces the frequency, rate or extent of ruffle assembly. Relationships: is a type of GO:0120033; is a type of regulation of ruffle assembly [GO:1900027]; negatively regulates ruffle assembly [GO:0097178] Sources: GOC:TermGenie, GOC:yaf Also known as: down regulation of membrane ruffle formation, down regulation of membrane ruffling, negative regulation of membrane ruffle formation, negative regulation of membrane ruffling, down regulation of ruffle assembly